regulation of transcytosis [GO:1904298] (biological process) Definition: Any process that modulates the frequency, rate or extent of transcytosis. References: PMID:9664076 Sources: GOC:TermGenie, GO_REF:0000058 Relationships: is a type of GO:0051239; is a type of GO:0060627; regulates transcytosis [GO:0045056] Subtypes: negative regulation of transcytosis [GO:1904299], positive regulation of transcytosis [GO:1904300]